{
  "gene_symbol": "MKKS",
  "term_label": "chaperone-mediated protein complex assembly",
  "term_id": "GO:0051131",
  "gene_name": "Molecular chaperone MKKS",
  "gene": "UniProtKB:Q9NPJ1"
}